{
  "term_label": "K48-linked deubiquitinase activity",
  "gene_name": "Ubiquitin carboxyl-terminal hydrolase MINDY-1",
  "term_id": "GO:1990380",
  "gene_symbol": "MINDY1",
  "gene": "UniProtKB:Q8N5J2"
}